{
  "gene_symbol": "TLE7",
  "gene_name": "Transducin-like enhancer protein 7",
  "term_label": "transcription corepressor activity",
  "term_id": "GO:0003714",
  "gene": "UniProtKB:A0A1W2PR48"
}